{
  "gene_symbol": "ABLIM3",
  "term_label": "stress fiber",
  "gene_name": "Actin-binding LIM protein 3",
  "term_id": "GO:0001725",
  "gene": "UniProtKB:O94929"
}